ribonuclease V activity [GO:0033901] (molecular function) Also known as: endoribonuclease V activity Relationships: is a type of RNA endonuclease activity producing 3'-phosphomonoesters, hydrolytic mechanism [GO:0016892] Definition: Catalysis of the hydrolysis of poly(A), forming oligoribonucleotides and ultimately 3'-AMP. Sources: EC:3.1.27.8